{
  "term_id": "UNKNOWN:0002",
  "term_label": "Unknown biological process",
  "gene_name": "Formiminotransferase N-terminal subdomain-containing protein",
  "gene": "UniProtKB:E5RQL4",
  "gene_symbol": "FTCDNL1"
}